{
  "gene_symbol": "UBAP2",
  "gene_name": "Ubiquitin-associated protein 2",
  "gene": "UniProtKB:Q5T6F2",
  "term_id": "GO:0005737",
  "term_label": "cytoplasm"
}